calcium-induced calcium release activity [GO:0048763] (molecular function) Subtypes: ryanodine-sensitive calcium-release channel activity [GO:0005219], calcium-induced calcium release activity involved in regulation of presynaptic cytosolic calcium ion concentration [GO:1905054], calcium-induced calcium release activity involved in regulation of postsynaptic cytosolic calcium ion concentration [GO:1905058] Definition: Enables transmembrane transfer of calcium ions from an intracellular store to the cytosol on induction by increased calcium concentration. Relationships: is a type of GO:0015278 References: PMID:2990997, PMID:8381210, PMID:8653752 Sources: GOC:jid, GOC:nln